{
  "gene_name": "Death domain-associated protein 6",
  "term_id": "GO:0042393",
  "gene": "UniProtKB:Q9UER7",
  "gene_symbol": "DAXX",
  "term_label": "histone binding"
}